{
  "gene_symbol": "CALM2",
  "gene_name": "Calmodulin-2",
  "term_label": "myelin sheath",
  "term_id": "GO:0043209",
  "gene": "UniProtKB:P0DP24"
}